{
  "gene_symbol": "LYPD1",
  "gene_name": "Ly6_PLAUR domain-containing protein 1",
  "gene": "UniProtKB:Q8N2G4",
  "term_id": "GO:0095500",
  "term_label": "acetylcholine receptor signaling pathway"
}